{
  "gene_symbol": "TK1",
  "gene": "UniProtKB:P04183",
  "term_id": "GO:0004797",
  "term_label": "thymidine kinase activity",
  "gene_name": "Thymidine kinase, cytosolic"
}